luteolin biosynthetic process [GO:0033511] (biological process) Definition: The chemical reactions and pathways resulting in the formation of luteolin, 2-(3,4-dihydroxyphenyl)-5,7-dihydroxy-4H-chromen-4-one. Relationships: is_a flavone biosynthetic process [GO:0051553] Sources: GOC:mah Also known as: luteolin anabolism, luteolin biosynthesis, luteolin formation, luteolin synthesis